negative regulation of mesenchymal stem cell differentiation [GO:2000740] (biological process) Definition: Any process that stops, prevents or reduces the frequency, rate or extent of mesenchymal stem cell differentiation. Sources: GOC:obol Relationships: is a type of negative regulation of stem cell differentiation [GO:2000737]; is a type of GO:2000739; negatively regulates mesenchymal stem cell differentiation [GO:0072497] Subtypes: negative regulation of amniotic stem cell differentiation [GO:2000798]